{
  "gene": "UniProtKB:Q9NPH2",
  "term_label": "inositol biosynthetic process",
  "gene_name": "Inositol-3-phosphate synthase 1",
  "term_id": "GO:0006021",
  "gene_symbol": "ISYNA1"
}